{
  "term_label": "nucleus",
  "term_id": "GO:0005634",
  "gene": "UniProtKB:Q7RTZ2",
  "gene_name": "Ubiquitin carboxyl-terminal hydrolase 17-like protein 1",
  "gene_symbol": "USP17L1"
}